{
  "gene_name": "Calcium-activated chloride channel regulator 2",
  "gene_symbol": "CLCA2",
  "gene": "UniProtKB:Q9UQC9",
  "term_id": "GO:0005886",
  "term_label": "plasma membrane"
}